{
  "gene_symbol": "RACGAP1",
  "gene": "UniProtKB:Q9H0H5",
  "term_id": "GO:0032154",
  "term_label": "cleavage furrow",
  "gene_name": "Rac GTPase-activating protein 1"
}